medial-Golgi-derived vesicle fusion with Golgi trans cisterna membrane [GO:1990672] (biological process) Definition: The joining of the lipid bilayer membrane around a medial-Golgi-derived vesicle to the lipid bilayer membrane around the Golgi trans cisterna. Vesicles are involved in anterograde transport. References: PMID:16038056, PMID:24119662 Sources: GOC:bhm Relationships: is a type of Golgi vesicle fusion to target membrane [GO:0048210]; is_a vesicle fusion with Golgi apparatus [GO:0048280]; is part of inter-Golgi cisterna vesicle-mediated transport [GO:0048219]